snRNA transcription [GO:0009301] (biological process) Definition: The synthesis of small nuclear RNA (snRNA) from a DNA template. Sources: GOC:jl, ISBN:0321000382 Relationships: is a type of DNA-templated transcription [GO:0006351]; is a type of snRNA metabolic process [GO:0016073] Subtypes: snRNA transcription by RNA polymerase II [GO:0042795], snRNA transcription by RNA polymerase III [GO:0042796]